{
  "gene_symbol": "LRRC37A3",
  "gene": "UniProtKB:O60309",
  "term_label": "Unknown cellular component",
  "gene_name": "Leucine-rich repeat-containing protein 37A3",
  "term_id": "UNKNOWN:0003"
}